{
  "term_label": "membrane",
  "gene_name": "Protein delta homolog 1",
  "term_id": "GO:0016020",
  "gene": "UniProtKB:P80370",
  "gene_symbol": "DLK1"
}